gluconokinase activity [GO:0046316] (molecular function) Sources: EC:2.7.1.12, RHEA:19433 Definition: Catalysis of the reaction: D-gluconate + ATP = 6-phospho-D-gluconate + ADP + 2 H+. Also known as: ATP:D-gluconate 6-phosphotransferase activity, gluconate kinase activity, gluconokinase (phosphorylating) Relationships: is a type of kinase activity [GO:0016301]; is_a GO:0016773